4-acetamido-4,6-dideoxy-D-galactose transferase activity [GO:0102031] (MF) Relationships: is a type of hexosyltransferase activity [GO:0016758] Definition: Catalysis of the reaction: dTDP-4-acetamido-4,6-dideoxy-alpha-D-galactose + beta-D-ManNAcA-(1->4)-alpha-D-GlcNAc-1-diphospho-ditrans,polycis-undecaprenol = H+ + alpha-D-FucNAc4-(1->4)-beta-D-ManNAcA-(1->4)-D-GlcNAc-undecaprenyl diphosphate + dTDP. Sources: EC:2.4.1.325, GOC:pz